{
  "gene_name": "Reticulophagy regulator 3",
  "gene": "UniProtKB:Q86VR2",
  "term_id": "UNKNOWN:0003",
  "term_label": "Unknown cellular component",
  "gene_symbol": "RETREG3"
}